deltoid tuberosity development [GO:0035993] (biological process) Relationships: is a type of anatomical structure development [GO:0048856]; is part of GO:0060173; is part of bone development [GO:0060348] Definition: The process whose specific outcome is the progression of the deltoid tuberosity over time, from its formation to the mature structure. The deltoid tuberosity is the region on the shaft of the humerus to which the deltoid muscle attaches. The deltoid tuberosity develops through endochondral ossification in a two-phase process; an initiating tendon-dependent phase, and a muscle-dependent growth phase. References: PMID:17567668 Sources: GOC:yaf, UBERON:0002498, Wikipedia:Deltoid_tuberosity